{
  "term_id": "GO:0006955",
  "gene_symbol": "IL1A",
  "term_label": "immune response",
  "gene_name": "Interleukin-1 alpha",
  "gene": "UniProtKB:P01583"
}